{
  "gene_symbol": "ILKAP",
  "gene": "UniProtKB:Q9H0C8",
  "gene_name": "Integrin-linked kinase-associated serine_threonine phosphatase 2C",
  "term_label": "Unknown cellular component",
  "term_id": "UNKNOWN:0003"
}